{
  "gene": "UniProtKB:Q9BSH3",
  "gene_symbol": "NICN1",
  "term_id": "UNKNOWN:0002",
  "gene_name": "Nicolin-1",
  "term_label": "Unknown biological process"
}